{
  "term_id": "GO:0005886",
  "term_label": "plasma membrane",
  "gene_name": "Semaphorin-6A",
  "gene_symbol": "SEMA6A",
  "gene": "UniProtKB:Q9H2E6"
}